{
  "gene_symbol": "SCAF1",
  "term_id": "UNKNOWN:0002",
  "gene": "UniProtKB:Q9H7N4",
  "gene_name": "Splicing factor, arginine_serine-rich 19",
  "term_label": "Unknown biological process"
}